{
  "term_id": "GO:0005102",
  "gene": "UniProtKB:Q2MKA7",
  "term_label": "signaling receptor binding",
  "gene_name": "R-spondin-1",
  "gene_symbol": "RSPO1"
}